{
  "gene": "UniProtKB:Q02246",
  "term_id": "GO:0045202",
  "term_label": "synapse",
  "gene_symbol": "CNTN2",
  "gene_name": "Contactin-2"
}